{
  "term_label": "immunoglobulin V(D)J recombination",
  "term_id": "GO:0033152",
  "gene": "UniProtKB:P78527",
  "gene_symbol": "PRKDC",
  "gene_name": "DNA-dependent protein kinase catalytic subunit"
}